{
  "gene_symbol": "FRMD8P1",
  "gene": "UniProtKB:Q9BZ68",
  "term_id": "GO:0090090",
  "gene_name": "Putative FERM domain-containing protein FRMD8P1",
  "term_label": "negative regulation of canonical Wnt signaling pathway"
}